{
  "term_label": "enzyme-substrate adaptor activity",
  "term_id": "GO:0140767",
  "gene_symbol": "CDC23",
  "gene_name": "Cell division cycle protein 23 homolog",
  "gene": "UniProtKB:Q9UJX2"
}